DNA polymerase processivity factor activity [GO:0030337] (molecular function) Relationships: is a type of GO:0008047; positively regulates DNA polymerase activity [GO:0034061] References: PMID:7903401, PMID:8087839 Sources: GOC:mah Definition: An enzyme regulator activity that increases the processivity of polymerization by DNA polymerase, by allowing the polymerase to move rapidly along DNA while remaining topologically bound to it. Also known as: processivity clamp, sliding clamp